{
  "term_label": "Unknown biological process",
  "gene_symbol": "HDGFL3",
  "term_id": "UNKNOWN:0002",
  "gene": "UniProtKB:Q9Y3E1",
  "gene_name": "Hepatoma-derived growth factor-related protein 3"
}